{
  "gene": "UniProtKB:Q6Q0C0",
  "gene_name": "E3 ubiquitin-protein ligase TRAF7",
  "term_label": "ubiquitin ligase complex",
  "gene_symbol": "TRAF7",
  "term_id": "GO:0000151"
}